axonemal basal plate assembly [GO:0062235] (BP) Definition: The aggregation, arrangement and bonding together of a set of components to form an axonemal basal plate. References: PMID:23352055, PMID:30810527 Also known as: basal plate assembly, axoneme basal plate assembly, axonemal basal plate formation Relationships: is_a cellular component assembly [GO:0022607]; BFO_0000050 axoneme assembly [GO:0035082]